{
  "gene_name": "POTE ankyrin domain family member E",
  "term_label": "axon",
  "gene_symbol": "POTEE",
  "gene": "UniProtKB:Q6S8J3",
  "term_id": "GO:0030424"
}